{
  "gene_name": "Apolipoprotein C-I",
  "gene": "UniProtKB:P02654",
  "term_id": "GO:0034364",
  "gene_symbol": "APOC1",
  "term_label": "high-density lipoprotein particle"
}